response to p-xylene [GO:1901500] (biological process) Sources: GOC:TermGenie, GOC:mengo_curators Definition: Any process that results in a change in state or activity of a cell or an organism (in terms of movement, secretion, enzyme production, gene expression, etc.) as a result of a p-xylene stimulus. Relationships: is a type of response to xylene [GO:1901501]